{
  "term_label": "extracellular space",
  "term_id": "GO:0005615",
  "gene_symbol": "DMKN",
  "gene": "UniProtKB:Q6E0U4",
  "gene_name": "Dermokine"
}